{
  "gene_name": "Kynurenine formamidase",
  "term_id": "UNKNOWN:0001",
  "gene_symbol": "AFMID",
  "gene": "UniProtKB:Q63HM1",
  "term_label": "Unknown molecular function"
}